{
  "gene_symbol": "ZSCAN4",
  "term_id": "UNKNOWN:0003",
  "term_label": "Unknown cellular component",
  "gene_name": "Zinc finger and SCAN domain-containing protein 4",
  "gene": "UniProtKB:Q8NAM6"
}